{
  "term_label": "immunoglobulin complex",
  "term_id": "GO:0019814",
  "gene_symbol": "IGKV1D-13",
  "gene_name": "Immunoglobulin kappa variable 1D-13",
  "gene": "UniProtKB:A0A0B4J2D9"
}